{
  "term_id": "GO:0000228",
  "gene_symbol": "SPO11",
  "gene": "UniProtKB:Q9Y5K1",
  "term_label": "nuclear chromosome",
  "gene_name": "Meiotic recombination protein SPO11"
}